{
  "gene": "UniProtKB:Q8TD47",
  "gene_name": "Small ribosomal subunit protein eS4, Y isoform 2",
  "term_label": "structural constituent of ribosome",
  "gene_symbol": "RPS4Y2",
  "term_id": "GO:0003735"
}